{
  "term_id": "UNKNOWN:0002",
  "term_label": "Unknown biological process",
  "gene": "UniProtKB:Q8IUH3",
  "gene_name": "RNA-binding protein 45",
  "gene_symbol": "RBM45"
}